{
  "term_id": "UNKNOWN:0002",
  "gene": "UniProtKB:Q8N0U2",
  "term_label": "Unknown biological process",
  "gene_symbol": "TMEM61",
  "gene_name": "Transmembrane protein 61"
}